response to insulin-like growth factor stimulus [GO:1990418] (BP) References: PMID:21932665 Definition: Any process that results in a change in state or activity of a cell or an organism (in terms of movement, secretion, enzyme production, gene expression, etc.) as a result of an insulin-like growth factor stimulus. Relationships: is a type of response to hormone [GO:0009725]